{
  "gene": "UniProtKB:Q08999",
  "term_label": "transcription regulator complex",
  "gene_symbol": "RBL2",
  "gene_name": "Retinoblastoma-like protein 2",
  "term_id": "GO:0005667"
}